{
  "term_id": "UNKNOWN:0001",
  "gene_symbol": "KRT222",
  "gene": "UniProtKB:Q8N1A0",
  "term_label": "Unknown molecular function",
  "gene_name": "Keratin-like protein KRT222"
}